{
  "term_label": "Unknown cellular component",
  "gene_name": "Harmonin-binding protein USHBP1",
  "gene": "UniProtKB:Q8N6Y0",
  "gene_symbol": "USHBP1",
  "term_id": "UNKNOWN:0003"
}